{
  "gene": "UniProtKB:Q9BZJ6",
  "term_id": "GO:0004930",
  "term_label": "G protein-coupled receptor activity",
  "gene_name": "Probable G-protein coupled receptor 63",
  "gene_symbol": "GPR63"
}